{
  "gene_symbol": "GSTK1",
  "gene": "UniProtKB:Q9Y2Q3",
  "term_id": "GO:0005739",
  "gene_name": "Glutathione S-transferase kappa 1",
  "term_label": "mitochondrion"
}